{
  "gene_symbol": "ABCB5",
  "gene": "UniProtKB:Q2M3G0",
  "term_label": "apical plasma membrane",
  "term_id": "GO:0016324",
  "gene_name": "ATP-binding cassette sub-family B member 5"
}